{
  "gene_name": "Unconventional prefoldin RPB5 interactor 1",
  "term_label": "negative regulation of intrinsic apoptotic signaling pathway",
  "term_id": "GO:2001243",
  "gene": "UniProtKB:O94763",
  "gene_symbol": "URI1"
}